{
  "term_id": "UNKNOWN:0001",
  "term_label": "Unknown molecular function",
  "gene_name": "Protein CUSTOS",
  "gene": "UniProtKB:Q96C57",
  "gene_symbol": "CUSTOS"
}